{
  "term_label": "Unknown molecular function",
  "gene": "UniProtKB:Q8TAD7",
  "term_id": "UNKNOWN:0001",
  "gene_name": "Overexpressed in colon carcinoma 1 protein",
  "gene_symbol": "OCC1"
}